stress granule assembly [GO:0034063] (biological process) Relationships: is_a membraneless organelle assembly [GO:0140694] Regulation: regulated by regulation of stress granule assembly [GO:0062028]; positively regulated by GO:0062029; negatively regulated by negative regulation of stress granule assembly [GO:0062030] Definition: The aggregation, arrangement and bonding together of proteins and RNA molecules to form a stress granule. Also known as: SG assembly References: PMID:17392519 Sources: GOC:mah